retinoid binding [GO:0005501] (MF) Definition: Binding to a retinoid, a class of isoprenoids that contain or are derived from four prenyl groups linked head-to-tail. Retinoids include retinol and retinal and structurally similar natural derivatives or synthetic compounds, but need not have vitamin A activity. Sources: GOC:jl, ISBN:0198506732 Relationships: is a type of isoprenoid binding [GO:0019840] Subtypes: retinoic acid binding [GO:0001972], retinal binding [GO:0016918], retinol binding [GO:0019841], GO:0046876